corticosteroid hormone secretion [GO:0035930] (biological process) Also known as: corticosteroid secretion Sources: GOC:sl Relationships: is a type of steroid hormone secretion [GO:0035929] Regulation: RO_0002211 by GO:2000846; negatively regulated by negative regulation of corticosteroid hormone secretion [GO:2000847]; positively regulated by positive regulation of corticosteroid hormone secretion [GO:2000848] Definition: The regulated release of any corticosteroid hormone into the circulatory system. Subtypes: mineralocorticoid secretion [GO:0035931], glucocorticoid secretion [GO:0035933]